{
  "gene_name": "Retinol dehydrogenase 10",
  "term_label": "Unknown biological process",
  "gene": "UniProtKB:Q8IZV5",
  "gene_symbol": "RDH10",
  "term_id": "UNKNOWN:0002"
}